{
  "gene_name": "Carnitine O-palmitoyltransferase 1, brain isoform",
  "term_id": "UNKNOWN:0001",
  "gene": "UniProtKB:Q8TCG5",
  "gene_symbol": "CPT1C",
  "term_label": "Unknown molecular function"
}